{
  "term_label": "positive regulation of phosphatidylinositol 3-kinase/protein kinase B signal transduction",
  "gene": "UniProtKB:Q8WYR1",
  "gene_name": "Phosphoinositide 3-kinase regulatory subunit 5",
  "term_id": "GO:0051897",
  "gene_symbol": "PIK3R5"
}